{
  "term_label": "male gonad development",
  "gene": "UniProtKB:Q13323",
  "gene_name": "Bcl-2-interacting killer",
  "gene_symbol": "BIK",
  "term_id": "GO:0008584"
}